meiosis II [GO:0007135] (biological process) Relationships: is a type of meiosis II cell cycle process [GO:0061983]; is a type of meiotic nuclear division [GO:0140013] Definition: The second nuclear division of meiosis, in which the two chromatids in each chromosome are separated, resulting in four daughter nuclei from the two nuclei produced in meiosis II. Also known as: meiosis II nuclear division Sources: GOC:dph, GOC:mah, ISBN:0198547684 Subtypes: male meiosis II [GO:0007142], female meiosis II [GO:0007147]